{
  "term_id": "GO:0005737",
  "gene_name": "Cdc42 effector protein 4",
  "gene": "UniProtKB:Q9H3Q1",
  "gene_symbol": "CDC42EP4",
  "term_label": "cytoplasm"
}